{
  "gene": "UniProtKB:Q5T7B8",
  "term_label": "microtubule depolymerization",
  "gene_name": "Kinesin-like protein KIF24",
  "term_id": "GO:0007019",
  "gene_symbol": "KIF24"
}